{
  "gene": "UniProtKB:Q02297",
  "gene_name": "Pro-neuregulin-1, membrane-bound isoform",
  "term_id": "GO:0038133",
  "term_label": "ERBB2-ERBB3 signaling pathway",
  "gene_symbol": "NRG1"
}